{
  "gene_symbol": "ODAD2",
  "term_id": "UNKNOWN:0003",
  "gene": "UniProtKB:Q5T2S8",
  "term_label": "Unknown cellular component",
  "gene_name": "Outer dynein arm-docking complex subunit 2"
}